positive regulation of abscisic acid biosynthetic process [GO:0010116] (biological process) Definition: Any process that activates or increases the frequency, rate or extent of the chemical reactions and pathways resulting in the formation of abscisic acid. Sources: GOC:sm Also known as: positive regulation of abscisic acid anabolism, positive regulation of abscisic acid biosynthesis, positive regulation of abscisic acid formation, positive regulation of abscisic acid synthesis, up regulation of abscisic acid biosynthetic process, up-regulation of abscisic acid biosynthetic process, upregulation of abscisic acid biosynthetic process, activation of abscisic acid biosynthetic process, stimulation of abscisic acid biosynthetic process Relationships: is a type of regulation of abscisic acid biosynthetic process [GO:0010115]; is a type of positive regulation of lipid biosynthetic process [GO:0046889]; is a type of GO:1902932; RO_0002213 GO:0009688